{
  "term_id": "GO:0006357",
  "gene_symbol": "ANKRD2",
  "term_label": "regulation of transcription by RNA polymerase II",
  "gene": "UniProtKB:Q9GZV1",
  "gene_name": "Ankyrin repeat domain-containing protein 2"
}